{
  "term_id": "UNKNOWN:0002",
  "gene": "UniProtKB:Q6ZQQ6",
  "gene_name": "WD repeat-containing protein 87",
  "term_label": "Unknown biological process",
  "gene_symbol": "WDR87"
}